{
  "gene_symbol": "LHFPL1",
  "term_label": "Unknown biological process",
  "gene": "UniProtKB:Q86WI0",
  "term_id": "UNKNOWN:0002",
  "gene_name": "LHFPL tetraspan subfamily member 1 protein"
}